{
  "term_id": "GO:0007156",
  "gene": "UniProtKB:P35613",
  "gene_symbol": "BSG",
  "term_label": "homophilic cell-cell adhesion",
  "gene_name": "Basigin"
}